{
  "gene_name": "Constitutive coactivator of PPAR-gamma-like protein 2",
  "gene": "UniProtKB:Q9NX05",
  "term_id": "GO:0005634",
  "term_label": "nucleus",
  "gene_symbol": "FAM120C"
}